{
  "gene_symbol": "SLC6A2",
  "gene_name": "Sodium-dependent noradrenaline transporter",
  "term_id": "GO:0015874",
  "term_label": "norepinephrine transport",
  "gene": "UniProtKB:P23975"
}